cytosol to ERGIC protein transport [GO:0106273] (biological process) References: PMID:32272059 Relationships: is a type of protein transport [GO:0015031] Definition: The directed movement of proteins from the cystosol to the endoplasmic reticulum-Golgi intermediate compartment (ERGIC).